symbiont-mediated suppression of host JAK-STAT cascade via inhibition of STAT activity [GO:0039562] (biological process) Definition: A process in which a symbiont interferes with, inhibits or disrupt a JAK-STAT signal cascade in the host organism by reducing the activity of host STAT (signal transducer and activator of transcription). STATs are SH2 domain-containing proteins which lie downstream of many signaling receptors. Upon phosphorylation by JAKs, STAT proteins hetero- or homo-dimerize and translocate to the nucleus to activate transcription of target genes. Subtypes: GO:0039563, symbiont-mediated suppression of host JAK-STAT cascade via inhibition of STAT2 activity [GO:0039564] Sources: GOC:bf Also known as: suppression by virus of host JAK-STAT cascade via inhibition of STAT activity, suppression by virus of host STAT activity, suppression by virus of host signal transducer and activator of transcription activity, disruption by virus of host JAK-STAT cascade via inhibition of STAT activity, inhibition by virus of host STAT activity Relationships: is a type of symbiont-mediated suppression of host JAK-STAT cascade [GO:0039514] Note: This term is for annotation of symbiont proteins that counteract the host innate immune response.